ADP phosphatase activity [GO:0043262] (molecular function) References: PMID:1470606 Sources: RHEA:61436 Definition: Catalysis of the reaction: ADP + H2O = AMP + phosphate + H+. Also known as: ADP diphosphatase activity, ADPase, adenosine-diphosphatase activity, ADPase activity, ATP diphosphohydrolase activity, ATP-diphosphatase activity, adenosine diphosphatase activity Relationships: is_a nucleoside diphosphate phosphatase activity [GO:0017110]